negative regulation of melanocyte differentiation [GO:0045635] (biological process) Definition: Any process that stops, prevents, or reduces the frequency, rate or extent of melanocyte differentiation. Relationships: is a type of regulation of melanocyte differentiation [GO:0045634]; is a type of negative regulation of pigment cell differentiation [GO:0050941]; negatively regulates melanocyte differentiation [GO:0030318] Subtypes: negative regulation of early stripe melanocyte differentiation [GO:0050947], negative regulation of late stripe melanocyte differentiation [GO:0050949] Also known as: down regulation of melanocyte differentiation, down-regulation of melanocyte differentiation, downregulation of melanocyte differentiation, negative regulation of melanophore differentiation, inhibition of melanocyte differentiation Sources: GOC:go_curators